type B pancreatic cell differentiation [GO:0003309] (biological process) Relationships: is a type of enteroendocrine cell differentiation [GO:0035883]; is part of endocrine pancreas development [GO:0031018] Also known as: pancreatic B cell differentiation, pancreatic beta cell differentiation Definition: The process in which relatively unspecialized cells acquire specialized structural and/or functional features of a type B pancreatic cell. A type B pancreatic cell is a cell located towards center of the islets of Langerhans that secretes insulin. References: PMID:11076772 Sources: CL:0000169, GOC:dph